mannosylfructose-phosphate synthase activity [GO:0103011] (molecular function) Relationships: is a type of hexosyltransferase activity [GO:0016758] Sources: EC:2.4.1.246, GOC:pz Definition: Catalysis of the reaction: GDP-alpha-D-mannose + beta-D-fructofuranose 6-phosphate = mannosylfructose-phosphate + GDP.